{
  "gene_name": "Zinc finger protein 20",
  "gene": "UniProtKB:P17024",
  "gene_symbol": "ZNF20",
  "term_label": "RNA polymerase II transcription regulatory region sequence-specific DNA binding",
  "term_id": "GO:0000977"
}